{
  "gene_name": "Putative keratin-associated protein 20-4",
  "term_label": "Unknown cellular component",
  "term_id": "UNKNOWN:0003",
  "gene": "UniProtKB:Q3LI62",
  "gene_symbol": "KRTAP20-4"
}